MyD88-independent toll-like receptor signaling pathway [GO:0002756] (BP) Also known as: MyD88-independent TLR signaling pathway, MyD88-independent toll-like receptor signalling pathway References: PMID:12467241, PMID:12524386, PMID:12855817, PMID:15585605, PMID:15728447 Sources: GOC:add, ISBN:0781735149 Regulation: regulated by GO:0034127; negatively regulated by negative regulation of MyD88-independent toll-like receptor signaling pathway [GO:0034128]; positively regulated by positive regulation of MyD88-independent toll-like receptor signaling pathway [GO:0034129] Relationships: is a type of toll-like receptor signaling pathway [GO:0002224] Definition: A toll-like receptor signaling pathway not relying on the MyD88 adaptor molecule. Toll-like receptors directly bind pattern motifs from a variety of microbial sources to initiate innate an immune response. Subtypes: TRIF-dependent toll-like receptor signaling pathway [GO:0035666], TRAM-dependent toll-like receptor signaling pathway [GO:0035668]